{
  "gene_name": "Zinc finger protein 20",
  "term_id": "GO:0000981",
  "gene_symbol": "ZNF20",
  "gene": "UniProtKB:P17024",
  "term_label": "DNA-binding transcription factor activity, RNA polymerase II-specific"
}